alphaV-beta3 integrin-laminin alpha-4 complex [GO:0071131] (cellular component) Relationships: is a type of plasma membrane protein complex [GO:0098797] Also known as: ITGAV-ITGB3-LAMA4 complex Definition: A protein complex that consists of an alphaV-beta3 integrin complex bound to laminin alpha-4. References: PMID:16824487